symbiont-mediated migration across host transepithelium [GO:0035756] (biological process) Relationships: is a type of symbiont-mediated migration across host tissue barrier [GO:0141142] Regulation: positively regulated by positive regulation of transepithelial migration of symbiont in host [GO:0140471] Definition: A process in which a symbiont moves from one side of an epithelium to the other within its host organism. The host is defined as the larger of the organisms involved in a symbiotic interaction. Also known as: migration in host through an epithelial cell layer, migration of symbiont within host by transepithelial trafficking, symbiont-mediated migration through host transepithelium, transepithelial migration of symbiont in host, transmigration of symbiont in host References: PMID:10639460 Sources: GOC:bf